formylmethanofuran dehydrogenase activity [GO:0018493] (molecular function) Definition: Catalysis of the reaction: N-formylmethanofuran + A + H2O + H+ = AH(2) + CO2 + methanofuran. Relationships: is a type of oxidoreductase activity, acting on the aldehyde or oxo group of donors [GO:0016903] Sources: EC:1.2.7.12, RHEA:19841 Also known as: formylmethanofuran:(acceptor) oxidoreductase activity, formylmethanofuran:acceptor oxidoreductase activity